{
  "term_label": "synaptic transmission, glutamatergic",
  "term_id": "GO:0035249",
  "gene_symbol": "NAPA",
  "gene": "UniProtKB:P54920",
  "gene_name": "Alpha-soluble NSF attachment protein"
}